{
  "term_label": "fibroblast growth factor receptor binding",
  "gene": "UniProtKB:Q9HCT0",
  "gene_symbol": "FGF22",
  "term_id": "GO:0005104",
  "gene_name": "Fibroblast growth factor 22"
}